{
  "gene_name": "Death effector domain-containing protein",
  "gene": "UniProtKB:O75618",
  "term_id": "GO:0003677",
  "term_label": "DNA binding",
  "gene_symbol": "DEDD"
}